{
  "gene": "UniProtKB:Q8IZF2",
  "term_label": "energy reserve metabolic process",
  "gene_symbol": "ADGRF5",
  "term_id": "GO:0006112",
  "gene_name": "Adhesion G protein-coupled receptor F5"
}